4-nitrophenol metabolic process [GO:0018960] (biological process) Definition: The chemical reactions and pathways involving 4-nitrophenol, a nitroaromatic compound which is used in the production of dyes, leather treatment agents, fungicides and as an intermediate in the production of the insecticide parathion. Sources: GOC:jl Also known as: 4-nitrophenol metabolism, p-nitrophenol metabolic process, p-nitrophenol metabolism Relationships: is a type of phenol-containing compound metabolic process [GO:0018958] Subtypes: 4-nitrophenol catabolic process [GO:0046196]